{
  "gene": "UniProtKB:Q8WUA8",
  "gene_name": "Tsukushi",
  "term_id": "UNKNOWN:0001",
  "term_label": "Unknown molecular function",
  "gene_symbol": "TSKU"
}